formate dehydrogenase (cytochrome) activity [GO:0047898] (molecular function) Sources: EC:1.2.2.1, MetaCyc:FORMATE-DEHYDROGENASE-CYTOCHROME-RXN Relationships: is a type of oxidoreductase activity, acting on the aldehyde or oxo group of donors, cytochrome as acceptor [GO:0016622] Definition: Catalysis of the reaction: formate + ferricytochrome b1 = CO2 + ferrocytochrome b1. Also known as: formate:cytochrome b1 oxidoreductase activity, formate:ferricytochrome-b1 oxidoreductase activity